{
  "term_id": "UNKNOWN:0001",
  "term_label": "Unknown molecular function",
  "gene_symbol": "TMEM186",
  "gene_name": "Transmembrane protein 186",
  "gene": "UniProtKB:Q96B77"
}